{
  "term_label": "retrograde transport, endosome to Golgi",
  "gene": "UniProtKB:Q6VEQ5",
  "gene_symbol": "WASH2P",
  "term_id": "GO:0042147",
  "gene_name": "WAS protein family homolog 2"
}